{
  "gene_name": "Serpin B9",
  "gene": "UniProtKB:P50453",
  "term_label": "extracellular space",
  "term_id": "GO:0005615",
  "gene_symbol": "SERPINB9"
}